{
  "gene_name": "Very-long-chain (3R)-3-hydroxyacyl-CoA dehydratase 1",
  "term_label": "endoplasmic reticulum membrane",
  "gene": "UniProtKB:B0YJ81",
  "gene_symbol": "HACD1",
  "term_id": "GO:0005789"
}